{
  "term_label": "Unknown molecular function",
  "gene_symbol": "MB21D2",
  "gene": "UniProtKB:Q8IYB1",
  "gene_name": "Nucleotidyltransferase MB21D2",
  "term_id": "UNKNOWN:0001"
}